{
  "term_label": "exocytosis",
  "gene": "UniProtKB:Q12829",
  "term_id": "GO:0006887",
  "gene_symbol": "RAB40B",
  "gene_name": "Ras-related protein Rab-40B"
}